{
  "gene": "UniProtKB:Q13105",
  "gene_symbol": "ZBTB17",
  "gene_name": "Zinc finger and BTB domain-containing protein 17",
  "term_label": "DNA-binding transcription repressor activity, RNA polymerase II-specific",
  "term_id": "GO:0001227"
}